{
  "term_label": "Unknown molecular function",
  "term_id": "UNKNOWN:0001",
  "gene_name": "Putative protein FAM90A5P",
  "gene_symbol": "FAM90A5P",
  "gene": "UniProtKB:A8MXJ8"
}